{
  "term_label": "nucleoplasm",
  "gene_symbol": "SPIN3",
  "gene": "UniProtKB:Q5JUX0",
  "term_id": "GO:0005654",
  "gene_name": "Spindlin-3"
}